{
  "gene": "UniProtKB:Q03135",
  "term_label": "regulation of cytosolic calcium ion concentration",
  "gene_symbol": "CAV1",
  "gene_name": "Caveolin-1",
  "term_id": "GO:0051480"
}